{
  "term_id": "GO:0005814",
  "gene_symbol": "CEP170",
  "gene_name": "Centrosomal protein of 170 kDa",
  "term_label": "centriole",
  "gene": "UniProtKB:Q5SW79"
}